regulation of teliospore formation [GO:0075256] (biological process) Definition: Any process that modulates the frequency, rate or extent of teliospore formation, which is the formation of a thick-walled resting or over-wintering spore produced by the rust fungi (Uredinales) and smut fungi (Ustilaginales) in which karyogamy occurs. Sources: GOC:pamgo_curators Relationships: is a type of regulation of asexual sporulation resulting in formation of a cellular spore [GO:0043943]; regulates teliospore formation [GO:0075255] Subtypes: positive regulation of teliospore formation [GO:0075257], negative regulation of teliospore formation [GO:0075258]